response to stem cell factor [GO:0036215] (biological process) Relationships: is_a GO:0034097 Also known as: response to KIT ligand, response to SCF, response to hematopoietic growth factor KL, response to stem cell factor stimulus Definition: Any process that results in a change in state or activity of a cell or an organism (in terms of movement, secretion, enzyme production, gene expression, etc.) as a result of a stem cell factor (SCF) stimulus. Subtypes: cellular response to stem cell factor stimulus [GO:0036216] Sources: GOC:uh